{
  "term_label": "Unknown biological process",
  "gene_name": "Neural cell adhesion molecule 1",
  "gene": "UniProtKB:P13591",
  "gene_symbol": "NCAM1",
  "term_id": "UNKNOWN:0002"
}